{
  "gene_symbol": "CDH12",
  "gene": "UniProtKB:P55289",
  "gene_name": "Cadherin-12",
  "term_label": "cell migration",
  "term_id": "GO:0016477"
}